{
  "term_label": "Unknown molecular function",
  "gene_name": "von Willebrand factor A domain-containing protein 1",
  "gene": "UniProtKB:Q6PCB0",
  "gene_symbol": "VWA1",
  "term_id": "UNKNOWN:0001"
}